{
  "gene_name": "Apolipoprotein A-I",
  "term_id": "GO:0033700",
  "gene_symbol": "APOA1",
  "gene": "UniProtKB:P02647",
  "term_label": "phospholipid efflux"
}